voltage-gated monoatomic ion channel activity involved in regulation of postsynaptic membrane potential [GO:1905030] (molecular function) Also known as: voltage-gated ion channel activity involved in regulation of postsynaptic membrane potential, voltage gated ion channel activity involved in regulation of post-synaptic membrane potential, voltage gated ion channel activity involved in regulation of postsynaptic membrane potential, voltage-dependent ion channel activity involved in regulation of post-synaptic membrane potential, voltage-dependent ion channel activity involved in regulation of postsynaptic membrane potential, voltage-gated ion channel activity involved in regulation of post-synaptic membrane potential Definition: Any voltage-gated ion channel activity that is involved in regulation of postsynaptic membrane potential. Relationships: is a type of voltage-gated monoatomic ion channel activity [GO:0005244]; is part of regulation of postsynaptic membrane potential [GO:0060078] Sources: GOC:TermGenie, GO_REF:0000061, ISBN:9780071120005